thioglucosidase binding [GO:0010180] (MF) Definition: Binding to a thioglucosidase enzyme. Sources: GOC:tb Also known as: myrosinase binding Relationships: is_a enzyme binding [GO:0019899]